cyanate biosynthetic process [GO:0046201] (biological process) Relationships: is a type of biosynthetic process [GO:0009058] Sources: GOC:ai Definition: The chemical reactions and pathways resulting in the formation of cyanate, NCO-, the anion of cyanic acid. Also known as: cyanate anabolism, cyanate biosynthesis, cyanate formation, cyanate synthesis